regulation of snRNA transcription by RNA polymerase II [GO:1905380] (biological process) Also known as: regulation of snRNA transcription from Pol II promoter, regulation of snRNA transcription from RNA polymerase II promoter Subtypes: negative regulation of snRNA transcription by RNA polymerase II [GO:1905381], positive regulation of snRNA transcription by RNA polymerase II [GO:1905382] Definition: Any process that modulates the frequency, rate or extent of snRNA transcription mediated by RNA polymerase II. References: PMID:10022900 Sources: GOC:TermGenie, GOC:bhm, GO_REF:0000058 Relationships: is a type of GO:0006357; regulates GO:0042795